negative regulation of cell growth involved in cardiac muscle cell development [GO:0061052] (biological process) Definition: Any process that decreases the rate, frequency, or extent of the growth of a cardiac muscle cell, where growth contributes to the progression of the cell over time from its initial formation to its mature state. Sources: GOC:dph Relationships: is a type of GO:0010614; is a type of negative regulation of cell growth [GO:0030308]; is a type of negative regulation of striated muscle cell differentiation [GO:0051154]; is a type of negative regulation of cardiac muscle tissue growth [GO:0055022]; is_a GO:0061050; negatively regulates GO:0061049